sodium-independent icosanoid transport [GO:0071718] (biological process) Sources: GOC:mah, GOC:sl Subtypes: sodium-independent leukotriene transport [GO:0071719], sodium-independent prostaglandin transport [GO:0071720], sodium-independent thromboxane transport [GO:0071721] Definition: The directed, sodium-independent, movement of icosanoids into, out of or within a cell, or between cells, by means of some agent such as a transporter or pore. Icosanoids are unsaturated C20 fatty acids and skeletally related compounds. Relationships: is a type of icosanoid transport [GO:0071715] Also known as: sodium-independent eicosanoid transport